{
  "gene_name": "COMM domain-containing protein 6",
  "gene_symbol": "COMMD6",
  "term_label": "NF-kappaB binding",
  "term_id": "GO:0051059",
  "gene": "UniProtKB:Q7Z4G1"
}